male gonad development [GO:0008584] (biological process) Also known as: testicular development, testis development Sources: GOC:jid Relationships: is_a GO:0008406; is part of development of primary male sexual characteristics [GO:0046546] Regulation: regulated by regulation of male gonad development [GO:2000018]; negatively regulated by negative regulation of male gonad development [GO:2000019]; positively regulated by GO:2000020 Definition: The process whose specific outcome is the progression of the male gonad over time, from its formation to the mature structure.